{
  "gene_name": "Coiled-coil domain-containing protein 113",
  "gene": "UniProtKB:Q9H0I3",
  "term_label": "ciliary basal body",
  "term_id": "GO:0036064",
  "gene_symbol": "CCDC113"
}